{
  "term_label": "cellular response to glucocorticoid stimulus",
  "gene_name": "UDP-glucuronosyltransferase 1A1",
  "gene_symbol": "UGT1A1",
  "term_id": "GO:0071385",
  "gene": "UniProtKB:P22309"
}